{
  "term_id": "GO:0005131",
  "gene_symbol": "GH1",
  "term_label": "growth hormone receptor binding",
  "gene": "UniProtKB:P01241",
  "gene_name": "Somatotropin"
}